{
  "gene_name": "Cytospin-A",
  "term_id": "GO:0031941",
  "gene_symbol": "SPECC1L",
  "term_label": "filamentous actin",
  "gene": "UniProtKB:Q69YQ0"
}